positive regulation of cytotoxic T cell degranulation [GO:0043319] (biological process) Definition: Any process that activates or increases the frequency, rate or extent of cytotoxic T cell degranulation. Relationships: is a type of GO:0001916; is a type of positive regulation of leukocyte degranulation [GO:0043302]; is a type of regulation of cytotoxic T cell degranulation [GO:0043317]; positively regulates GO:0043316 Sources: ISBN:0781735149 Also known as: positive regulation of cytotoxic T cell granule exocytosis, positive regulation of cytotoxic T lymphocyte degranulation, positive regulation of cytotoxic T lymphocyte granule exocytosis, positive regulation of cytotoxic T-cell degranulation, positive regulation of cytotoxic T-cell granule exocytosis, positive regulation of cytotoxic T-lymphocyte degranulation, positive regulation of cytotoxic T-lymphocyte granule exocytosis, up regulation of cytotoxic T cell degranulation, up-regulation of cytotoxic T cell degranulation, upregulation of cytotoxic T cell degranulation, activation of cytotoxic T cell degranulation, stimulation of cytotoxic T cell degranulation